{
  "gene_symbol": "OR2A25",
  "gene": "UniProtKB:A4D2G3",
  "gene_name": "Olfactory receptor 2A25",
  "term_id": "GO:0016020",
  "term_label": "membrane"
}